response to carbon dioxide [GO:0010037] (BP) Definition: Any process that results in a change in state or activity of a cell or an organism (in terms of movement, secretion, enzyme production, gene expression, etc.) as a result of a carbon dioxide (CO2) stimulus. Sources: GOC:sm Relationships: is a type of response to oxygen-containing compound [GO:1901700] Subtypes: cellular response to carbon dioxide [GO:0071244]